porin activity [GO:0015288] (molecular function) Subtypes: toxin export channel activity [GO:0000269], GO:0015471, GO:0015473, autotransporter activity [GO:0015474], oligosaccharide transporting porin activity [GO:0015478], maltose transporting porin activity [GO:0015481], long-chain fatty acid transporting porin activity [GO:0015483] Also known as: porin, outer membrane exporter porin Definition: Enables the transfer of substances, sized less than 1000 Da, from one side of a membrane to the other. The transmembrane portions of porins consist exclusively of beta-strands which form a beta-barrel. They are found in the outer membranes of Gram-negative bacteria, mitochondria, plastids and possibly acid-fast Gram-positive bacteria. Relationships: is a type of wide pore channel activity [GO:0022829] References: PMID:10839820 Sources: GOC:mtg_transport, ISBN:0815340729, TC:1.B.1.-.-